{
  "gene_name": "Amphiregulin",
  "term_label": "extracellular space",
  "gene": "UniProtKB:P15514",
  "term_id": "GO:0005615",
  "gene_symbol": "AREG"
}